UDP-alpha-D-glucose metabolic process [GO:0006011] (biological process) Also known as: UDP-glucose metabolism Subtypes: UDP-glucosylation [GO:0097359], UDP-alpha-D-glucose biosynthetic process [GO:0120530] Sources: GOC:ai Relationships: is a type of nucleotide-sugar metabolic process [GO:0009225] Definition: The chemical reactions and pathways involving UDP-alpha-D-glucose, a substance composed of alpha-D-glucose in glycosidic linkage with uridine diphosphate.